ergothioneine biosynthetic process [GO:0052699] (biological process) Definition: The chemical reactions and pathways resulting in the formation of ergothioneine, a naturally occurring metabolite of histidine with antioxidant properties. Sources: Wikipedia:Ergothioneine Also known as: (2S)-3-(2-mercapto-1H-imidazol-5-yl)-2-(trimethylazaniumyl)propanoate biosynthetic process, 2-mercaptoergothioneine trimethylbetaine anabolism, 2-mercaptoergothioneine trimethylbetaine biosynthesis, 2-mercaptoergothioneine trimethylbetaine biosynthetic process, 2-mercaptoergothioneine trimethylbetaine formation, 2-mercaptoergothioneine trimethylbetaine synthesis, ergothioneine anabolism, ergothioneine biosynthesis, ergothioneine formation, ergothioneine synthesis Relationships: is a type of sulfur amino acid biosynthetic process [GO:0000097]; is a type of amino-acid betaine biosynthetic process [GO:0006578]; is_a GO:0052698; is a type of modified histidine biosynthetic process [GO:0052703] Subtypes: ergothioneine biosynthesis from histidine via gamma-glutamyl-hercynylcysteine sulfoxide [GO:0052704], ergothioneine biosynthesis from histidine via hercynylcysteine sulfoxide synthase [GO:0140479]